oxidoreductase activity, acting on paired donors, with incorporation or reduction of molecular oxygen [GO:0016705] (molecular function) Subtypes: cholesterol 25-hydroxylase activity [GO:0001567], GO:0004501, GO:0004666, GO:0008387, steroid 15-alpha-hydroxylase activity [GO:0008388], GO:0008389, GO:0008391, GO:0008401, 25-hydroxycholecalciferol-24-hydroxylase activity [GO:0008403], 3-demethoxyubiquinol 3-hydroxylase activity [GO:0008682], 2-oxoglutarate-dependent dioxygenase activity [GO:0016706], oxidoreductase activity, acting on paired donors, with incorporation or reduction of molecular oxygen, NAD(P)H as one donor, and incorporation of two atoms of oxygen into one donor [GO:0016708], GO:0016709, oxidoreductase activity, acting on paired donors, with incorporation or reduction of molecular oxygen, reduced flavin or flavoprotein as one donor, and incorporation of one atom of oxygen [GO:0016712], oxidoreductase activity, acting on paired donors, with incorporation or reduction of molecular oxygen, reduced iron-sulfur protein as one donor, and incorporation of one atom of oxygen [GO:0016713], oxidoreductase activity, acting on paired donors, with incorporation or reduction of molecular oxygen, reduced pteridine as one donor, and incorporation of one atom of oxygen [GO:0016714], oxidoreductase activity, acting on paired donors, with incorporation or reduction of molecular oxygen, reduced ascorbate as one donor, and incorporation of one atom of oxygen [GO:0016715], oxidoreductase activity, acting on paired donors, with incorporation or reduction of molecular oxygen, another compound as one donor, and incorporation of one atom of oxygen [GO:0016716], oxidoreductase activity, acting on paired donors, with oxidation of a pair of donors resulting in the reduction of molecular oxygen to two molecules of water [GO:0016717], GO:0018597, 4-methoxybenzoate monooxygenase (O-demethylating) activity [GO:0018690], deoxyhypusine monooxygenase activity [GO:0019135], omega-3 fatty acid desaturase activity [GO:0042389], gamma-glutamyl hercynylcysteine sulfoxide synthase activity [GO:0044875], GO:0045301, omega-6 fatty acid desaturase activity [GO:0045485], phylloquinone monooxygenase (2,3-epoxidizing) activity [GO:0047097], Latia-luciferin monooxygenase (demethylating) activity [GO:0047098], GO:0047546, 3-hydroxybenzoate 2-monooxygenase activity [GO:0047563], estradiol 6-beta-monooxygenase activity [GO:0047882], kynurenine 7,8-hydroxylase activity [GO:0050016], progesterone monooxygenase activity [GO:0050214], steroid 9-alpha-monooxygenase activity [GO:0050292], oxidoreductase activity, acting on paired donors, with incorporation or reduction of molecular oxygen, with 2-oxoglutarate as one donor, and the other dehydrogenated [GO:0050498], thiophene-2-carbonyl-CoA monooxygenase activity [GO:0050603], GO:0050604, uracil oxygenase activity [GO:0052614], all-trans retinol 3,4-desaturase activity [GO:0061896], GO:0061897, all-trans retinoic acid 3,4-desaturase activity [GO:0061898], 11-cis-retinal 3,4-desaturase activity [GO:0061899], GO:0062146, amorpha-4,11-diene 12-monooxygenase activity [GO:0062150], linoleic acid epoxygenase activity [GO:0071614], thalian-diol desaturase activity [GO:0080004], GO:0080102, 4-methylthiopropyl glucosinolate S-oxygenase activity [GO:0080103], 5-methylthiopropyl glucosinolate S-oxygenase activity [GO:0080104], 6-methylthiopropyl glucosinolate S-oxygenase activity [GO:0080105], 7-methylthiopropyl glucosinolate S-oxygenase activity [GO:0080106], 8-methylthiopropyl glucosinolate S-oxygenase activity [GO:0080107], 11alpha-30-dihydroxy beta-amyrin dehydrogenase activity [GO:0102369], typhasterol C-23 hydroxylase activity [GO:0102733], methylcytosine to 5-glyceryl-methylcytosine dioxygenase activity [GO:0120204], GO:0140395, FAD-dependent H3K4me/H3K4me3 demethylase activity [GO:0140682], FAD-dependent histone H3K9me/H3K9me2 demethylase activity [GO:0140685], halogenase activity [GO:0140906] Also known as: oxidoreductase activity, acting on paired donors, with incorporation or reduction of molecular oxygen, miscellaneous Sources: EC:1.14.-.- Definition: Catalysis of an oxidation-reduction (redox) reaction in which hydrogen or electrons are transferred from each of two donors, and molecular oxygen is reduced or incorporated into a donor. Relationships: is a type of GO:0016491